{
  "term_id": "UNKNOWN:0001",
  "term_label": "Unknown molecular function",
  "gene_symbol": "ERRFI1",
  "gene": "UniProtKB:Q9UJM3",
  "gene_name": "ERBB receptor feedback inhibitor 1"
}